{
  "term_label": "phosphatidylinositol-4-phosphate binding",
  "term_id": "GO:0070273",
  "gene_symbol": "GSDMA",
  "gene_name": "Gasdermin-A",
  "gene": "UniProtKB:Q96QA5"
}